{
  "gene_name": "Protein Jade-1",
  "term_label": "chromatin remodeling",
  "gene": "UniProtKB:Q6IE81",
  "gene_symbol": "JADE1",
  "term_id": "GO:0006338"
}